PCNA complex [GO:0043626] (cellular component) Definition: A protein complex composed of three identical PCNA monomers, each comprising two similar domains, which are joined in a head-to-tail arrangement to form a homotrimer. Forms a ring-like structure in solution, with a central hole sufficiently large to accommodate the double helix of DNA. Originally characterized as a DNA sliding clamp for replicative DNA polymerases and as an essential component of the replisome, and has also been shown to be involved in other processes including Okazaki fragment processing, DNA repair, translesion DNA synthesis, DNA methylation, chromatin remodeling and cell cycle regulation. References: PMID:12829735 Sources: GOC:jl Also known as: sliding clamp, PCNA homotrimer, proliferating cell nuclear antigen complex Relationships: is a type of DNA polymerase processivity factor complex [GO:0044796]; is a type of nuclear protein-containing complex [GO:0140513]